embryonic meristem development [GO:0048508] (biological process) Sources: GOC:jid Relationships: is a type of developmental process involved in reproduction [GO:0003006]; is a type of meristem development [GO:0048507]; is part of GO:0009793 Definition: The process whose specific outcome is the progression of the embryonic meristem over time, from its formation to the mature structure. Subtypes: primary meristem tissue development [GO:0010065]